positive regulation of plant-type cell wall cellulose biosynthetic process [GO:2001011] (biological process) Also known as: positive regulation of cell wall cellulose biosynthesis, positive regulation of cellulose biosynthesis during cell wall biosynthesis Definition: Any process that activates or increases the frequency, rate or extent of plant-type cell wall cellulose biosynthetic process. Relationships: is a type of positive regulation of cellular component biogenesis [GO:0044089]; is a type of positive regulation of cellulose biosynthetic process [GO:2001008]; is a type of regulation of plant-type cell wall cellulose biosynthetic process [GO:2001009]; positively regulates plant-type cell wall cellulose biosynthetic process [GO:0052324] Sources: GOC:mengo_curators